cell redox homeostasis [GO:0045454] (biological process) References: PMID:38689066 Sources: GOC:ai, GOC:dph, GOC:tb Definition: Any process that maintains the redox environment of a cell or compartment within a cell. Relationships: is a type of cellular homeostasis [GO:0019725] Also known as: regulation of redox homeostasis, regulation of cell redox homeostasis